{
  "gene_name": "Mannosyl-oligosaccharide 1,2-alpha-mannosidase IB",
  "gene": "UniProtKB:O60476",
  "term_label": "mannosyl-oligosaccharide 1,2-alpha-mannosidase activity",
  "gene_symbol": "MAN1A2",
  "term_id": "GO:0004571"
}